cerebral cortex tangential migration [GO:0021800] (biological process) Definition: The migration of cells in the cerebral cortex in which cells move orthogonally to the direction of radial migration and do not use radial glial cell processes as substrates for migration. References: PMID:12626695 Sources: GOC:cls, GOC:dgh, GOC:dph, GOC:jid, GO_REF:0000021 Relationships: is a type of GO:0021795 Subtypes: substrate-dependent cerebral cortex tangential migration [GO:0021825]